{
  "gene_name": "Baculoviral IAP repeat-containing protein 7",
  "gene_symbol": "BIRC7",
  "term_label": "positive regulation of protein ubiquitination",
  "gene": "UniProtKB:Q96CA5",
  "term_id": "GO:0031398"
}